{
  "gene_symbol": "OR2M4",
  "term_id": "GO:0004984",
  "gene": "UniProtKB:Q96R27",
  "term_label": "olfactory receptor activity",
  "gene_name": "Olfactory receptor 2M4"
}